convergent extension involved in mesonephric nephron morphogenesis [GO:0061237] (biological process) Definition: The morphogenetic process in which the renal epithelium narrows along one axis and lengthens in a perpendicular axis that contributes to the shaping of a nephron in the mesonephros. Relationships: is a type of GO:0072045; is part of GO:0061228 Sources: GOC:mtg_kidney_jan10